regulation of cell migration [GO:0030334] (biological process) Relationships: is a type of regulation of cell motility [GO:2000145]; regulates cell migration [GO:0016477] Subtypes: regulation of leukocyte migration [GO:0002685], regulation of endothelial cell migration [GO:0010594], regulation of epithelial cell migration [GO:0010632], regulation of fibroblast migration [GO:0010762], regulation of smooth muscle cell migration [GO:0014910], directional guidance of interneurons involved in migration from the subpallium to the cortex [GO:0021840], neurotransmitter-mediated guidance of interneurons involved in substrate-independent cerebral cortex tangential migration [GO:0021845], GO:0030335, negative regulation of cell migration [GO:0030336], regulation of angioblast cell migration involved in selective angioblast sprouting [GO:0035477], regulation of neuroblast migration [GO:0061853], regulation of cell migration involved in somitogenic axis elongation [GO:0090249], regulation of myotube cell migration [GO:0110123], regulation of trophoblast cell migration [GO:1901163], regulation of distal tip cell migration [GO:1903354], regulation of wound healing, spreading of epidermal cells [GO:1903689], regulation of glial cell migration [GO:1903975], GO:1904235, regulation of cell chemotaxis to fibroblast growth factor [GO:1904847], regulation of endothelial cell chemotaxis to vascular endothelial growth factor [GO:1904857], GO:1905210, regulation of cardiac neural crest cell migration involved in outflow tract morphogenesis [GO:1905310], regulation of mesenchymal stem cell migration [GO:1905320], regulation of hematopoietic stem cell migration [GO:2000471], regulation of metanephric mesenchymal cell migration [GO:2000589], regulation of neuron migration [GO:2001222], GO:2001281 Definition: Any process that modulates the frequency, rate or extent of cell migration. Sources: GOC:go_curators